{
  "gene": "UniProtKB:Q9NRB3",
  "term_label": "Unknown cellular component",
  "gene_symbol": "CHST12",
  "term_id": "UNKNOWN:0003",
  "gene_name": "Carbohydrate sulfotransferase 12"
}